{
  "term_label": "Unknown molecular function",
  "term_id": "UNKNOWN:0001",
  "gene_name": "HOXB-AS3 peptide",
  "gene_symbol": "HOXB-AS3",
  "gene": "UniProtKB:C0HLZ6"
}